stereocilia tip-link density [GO:1990427] (cellular component) References: PMID:19447093, PMID:21709241 Definition: An electron-dense plaque at either end of a stereocilia tip link that provides the anchor in the stereocilia membrane. Subtypes: lower tip-link density [GO:1990434], upper tip-link density [GO:1990435] Relationships: is a type of cellular anatomical structure [GO:0110165]; is part of stereocilia tip link [GO:0002140]; is part of cell projection [GO:0042995]